regulation of telomeric loop formation [GO:1904418] (BP) Definition: Any process that modulates the frequency, rate or extent of telomeric loop formation. References: PMID:22579284 Sources: GOC:BHF, GOC:BHF_telomere, GOC:TermGenie, GOC:nc, GO_REF:0000058 Also known as: regulation of t-loop biosynthesis, regulation of t-loop formation Relationships: is a type of regulation of telomere maintenance [GO:0032204]; regulates telomeric loop formation [GO:0031627] Subtypes: negative regulation of telomeric loop formation [GO:1904419], positive regulation of telomeric loop formation [GO:1904420]